{
  "gene_symbol": "RNH1",
  "term_id": "GO:0034315",
  "term_label": "regulation of Arp2/3 complex-mediated actin nucleation",
  "gene_name": "Ribonuclease inhibitor",
  "gene": "UniProtKB:P13489"
}